{
  "gene": "UniProtKB:P37198",
  "gene_name": "Nuclear pore glycoprotein p62",
  "gene_symbol": "NUP62",
  "term_label": "structural constituent of nuclear pore",
  "term_id": "GO:0017056"
}